{
  "gene_symbol": "ZNF671",
  "gene": "UniProtKB:Q8TAW3",
  "term_id": "UNKNOWN:0003",
  "gene_name": "Zinc finger protein 671",
  "term_label": "Unknown cellular component"
}